{
  "gene": "UniProtKB:P49715",
  "term_id": "GO:0006357",
  "gene_symbol": "CEBPA",
  "gene_name": "CCAAT_enhancer-binding protein alpha",
  "term_label": "regulation of transcription by RNA polymerase II"
}